{
  "term_id": "GO:0070936",
  "gene_name": "Ubiquitin-conjugating enzyme E2 D2",
  "term_label": "protein K48-linked ubiquitination",
  "gene": "UniProtKB:P62837",
  "gene_symbol": "UBE2D2"
}